{
  "gene_name": "ERI1 exoribonuclease 2",
  "gene_symbol": "ERI2",
  "gene": "UniProtKB:A8K979",
  "term_id": "GO:0000175",
  "term_label": "3'-5'-RNA exonuclease activity"
}